establishment of integrated proviral latency [GO:0075713] (biological process) Definition: A process by which the virus integrates into the host genome and establishes as a stable provirus or prophage. Sources: GOC:jl Also known as: prophage integration, provirus integration Relationships: is a type of establishment of viral latency [GO:0019043]; BFO_0000051 viral genome integration into host DNA [GO:0044826]